{
  "gene_symbol": "SELL",
  "term_id": "GO:0009897",
  "term_label": "external side of plasma membrane",
  "gene_name": "L-selectin",
  "gene": "UniProtKB:P14151"
}